CAT tailing [GO:0140708] (biological process) Relationships: is a type of GO:0002182; is part of rescue of stalled ribosome [GO:0072344]; BFO_0000050 ribosome-associated ubiquitin-dependent protein catabolic process [GO:1990116] References: PMID:25554787, PMID:32934225 Definition: The C-terminal elongation of 60S-anchored stalled nascent polypeptide chains with untemplated alanine and threonine tails (CAT tails). CAT tails participate in the recognition of stalled nascent chains by the ribosome quality control system.